hexulose-6-phosphate synthase activity [GO:0043801] (molecular function) Definition: Catalysis of the reaction: D-ribulose 5-phosphate + formaldehyde = D-arabino-3-hexulose 6-phosphate. References: PMID:16075199 Relationships: is a type of GO:0016832